{
  "gene_symbol": "CHD7",
  "term_label": "nucleus",
  "gene_name": "Chromodomain-helicase-DNA-binding protein 7",
  "term_id": "GO:0005634",
  "gene": "UniProtKB:Q9P2D1"
}